negative regulation of promoter clearance from RNA polymerase II promoter [GO:0140847] (biological process) References: PMID:28248323 Definition: A process that stops, prevents or reduces the transition from the initiation to the elongation phases of transcription by RNA polymerase II. Relationships: is a type of regulation of promoter clearance from RNA polymerase II promoter [GO:0140845]; is a type of negative regulation of RNA biosynthetic process [GO:1902679]; negatively regulates RNA polymerase II promoter clearance [GO:0001111]